{
  "term_id": "UNKNOWN:0003",
  "gene_symbol": "DNER",
  "term_label": "Unknown cellular component",
  "gene": "UniProtKB:Q8NFT8",
  "gene_name": "Delta and Notch-like epidermal growth factor-related receptor"
}